{
  "gene_name": "Uncharacterized protein ARIH2OS",
  "gene": "UniProtKB:Q8N7S6",
  "term_id": "UNKNOWN:0003",
  "gene_symbol": "ARIH2OS",
  "term_label": "Unknown cellular component"
}